amide binding [GO:0033218] (molecular function) Sources: GOC:mah Definition: Binding to an amide, any derivative of an oxoacid in which an acidic hydroxy group has been replaced by an amino or substituted amino group. Relationships: is_a GO:0005488 Subtypes: GO:0001540, FK506 binding [GO:0005528], GO:0005542, penicillin binding [GO:0008658], biotin binding [GO:0009374], N-1-naphthylphthalamic acid binding [GO:0010013], cyclosporin A binding [GO:0016018], peptide hormone binding [GO:0017046], phosphopantetheine binding [GO:0031177], GO:0031626, muramyl dipeptide binding [GO:0032500], urea binding [GO:0033219], GO:0043544, suramin binding [GO:0043924], methotrexate binding [GO:0051870], GO:0071723, ceramide binding [GO:0097001], coenzyme A binding [GO:0120225], acyl-CoA binding [GO:0120227], oligopeptide binding [GO:1900750], dethiobiotin binding [GO:1901602], melatonin binding [GO:1904408]